{
  "gene_name": "Protein FAM106C",
  "term_id": "UNKNOWN:0001",
  "term_label": "Unknown molecular function",
  "gene_symbol": "FAM106C",
  "gene": "UniProtKB:P0CH98"
}